{
  "gene_symbol": "PM20D1",
  "gene_name": "N-fatty-acyl-amino acid synthase_hydrolase PM20D1",
  "gene": "UniProtKB:Q6GTS8",
  "term_label": "Unknown cellular component",
  "term_id": "UNKNOWN:0003"
}